regulation of dendritic cell apoptotic process [GO:2000668] (biological process) Sources: GOC:mtg_apoptosis, GOC:obol Definition: Any process that modulates the frequency, rate or extent of dendritic cell apoptotic process. Also known as: regulation of dendritic cell apoptosis Relationships: is a type of regulation of leukocyte apoptotic process [GO:2000106]; regulates dendritic cell apoptotic process [GO:0097048] Subtypes: negative regulation of dendritic cell apoptotic process [GO:2000669], positive regulation of dendritic cell apoptotic process [GO:2000670]